{
  "gene": "UniProtKB:Q9P2R6",
  "term_id": "GO:0005634",
  "gene_name": "Arginine-glutamic acid dipeptide repeats protein",
  "term_label": "nucleus",
  "gene_symbol": "RERE"
}